{
  "term_label": "Unknown cellular component",
  "gene": "UniProtKB:Q6VY07",
  "gene_symbol": "PACS1",
  "gene_name": "Phosphofurin acidic cluster sorting protein 1",
  "term_id": "UNKNOWN:0003"
}